{
  "term_label": "protein tyrosine kinase activity",
  "gene_symbol": "FER",
  "term_id": "GO:0004713",
  "gene": "UniProtKB:P16591",
  "gene_name": "Tyrosine-protein kinase Fer"
}